{
  "gene_name": "Beclin-1",
  "term_label": "protein-macromolecule adaptor activity",
  "gene_symbol": "BECN1",
  "term_id": "GO:0030674",
  "gene": "UniProtKB:Q14457"
}